{
  "term_id": "GO:0004568",
  "gene": "UniProtKB:Q01459",
  "gene_name": "Di-N-acetylchitobiase",
  "term_label": "chitinase activity",
  "gene_symbol": "CTBS"
}